{
  "gene_name": "Keratin-associated protein 1-1",
  "term_label": "Unknown cellular component",
  "gene_symbol": "KRTAP1-1",
  "term_id": "UNKNOWN:0003",
  "gene": "UniProtKB:Q07627"
}